{
  "gene_name": "HIV Tat-specific factor 1",
  "gene": "UniProtKB:O43719",
  "gene_symbol": "HTATSF1",
  "term_label": "Unknown biological process",
  "term_id": "UNKNOWN:0002"
}